genitalia development [GO:0048806] (biological process) Also known as: genital development Sources: GOC:jid Subtypes: imaginal disc-derived genitalia development [GO:0007484], GO:0030539, GO:0030540 Definition: The process whose specific outcome is the progression of the genitalia over time, from its formation to the mature structure. Relationships: is_a animal organ development [GO:0048513]; is a type of GO:0048608; is part of sex differentiation [GO:0007548]